{
  "gene_name": "Homeobox protein Hox-D13",
  "gene_symbol": "HOXD13",
  "term_id": "GO:0000978",
  "gene": "UniProtKB:P35453",
  "term_label": "RNA polymerase II cis-regulatory region sequence-specific DNA binding"
}